{
  "term_id": "UNKNOWN:0003",
  "term_label": "Unknown cellular component",
  "gene_symbol": "FAM240B",
  "gene_name": "Protein FAM240B",
  "gene": "UniProtKB:A0A1B0GVZ2"
}